{
  "gene_symbol": "LRIG3",
  "term_id": "GO:0038023",
  "gene": "UniProtKB:Q6UXM1",
  "gene_name": "Leucine-rich repeats and immunoglobulin-like domains protein 3",
  "term_label": "signaling receptor activity"
}